{
  "term_id": "UNKNOWN:0003",
  "gene": "UniProtKB:Q9Y5Q6",
  "gene_name": "Insulin-like peptide INSL5",
  "term_label": "Unknown cellular component",
  "gene_symbol": "INSL5"
}